{
  "gene": "UniProtKB:A8MWP4",
  "term_label": "Unknown molecular function",
  "gene_symbol": "A8MWP4",
  "gene_name": "Putative uncharacterized protein ENSP00000401716",
  "term_id": "UNKNOWN:0001"
}